{
  "gene_symbol": "STMN4",
  "term_label": "regulation of microtubule polymerization or depolymerization",
  "gene_name": "Stathmin-4",
  "gene": "UniProtKB:Q9H169",
  "term_id": "GO:0031110"
}